{
  "term_id": "GO:0000122",
  "gene_name": "B-cell CLL_lymphoma 6 member B protein",
  "term_label": "negative regulation of transcription by RNA polymerase II",
  "gene_symbol": "BCL6B",
  "gene": "UniProtKB:Q8N143"
}